{
  "term_id": "GO:0000978",
  "gene_name": "Nuclear transcription factor Y subunit beta",
  "gene": "UniProtKB:P25208",
  "gene_symbol": "NFYB",
  "term_label": "RNA polymerase II cis-regulatory region sequence-specific DNA binding"
}